cysteine lyase activity [GO:0047803] (molecular function) Sources: EC:4.4.1.10, MetaCyc:CYSTEINE-LYASE-RXN Definition: Catalysis of the reaction: L-cysteine + sulfite = L-cysteate + sulfide. Relationships: is a type of carbon-sulfur lyase activity [GO:0016846] Also known as: L-cysteine hydrogen-sulfide-lyase (adding sulfite), L-cysteine hydrogen-sulfide-lyase (adding sulfite; L-cysteate-forming), cysteine (sulfite) lyase activity